{
  "gene_name": "Transcription elongation regulator 1",
  "gene_symbol": "TCERG1",
  "gene": "UniProtKB:O14776",
  "term_label": "RNA polymerase binding",
  "term_id": "GO:0070063"
}